{
  "gene": "UniProtKB:Q9UBD0",
  "term_id": "GO:0003700",
  "term_label": "DNA-binding transcription factor activity",
  "gene_name": "Heat shock transcription factor, X-linked",
  "gene_symbol": "HSFX2"
}